Notch receptor processing, ligand-dependent [GO:0035333] (biological process) Also known as: Notch S2 cleavage, Notch S3 cleavage Definition: The proteolytic cleavages to the Notch protein that occur as a result of ligand binding. Ligand binding at the cell surface exposes an otherwise inaccessible cleavage site in the extracellular portion of Notch, which when cleaved releases a membrane-tethered form of the Notch intracellular domain. Subsequent cleavage within the transmembrane domain then leads to the release of the soluble Notch intracellular domain (NICD). Relationships: is_a membrane protein intracellular domain proteolysis [GO:0031293]; BFO_0000050 Notch signaling pathway [GO:0007219]; is part of Notch receptor processing [GO:0007220] References: PMID:12651094 Sources: GOC:bf